ribitol 2-dehydrogenase (NAD+) activity [GO:0050255] (molecular function) Definition: Catalysis of the reaction: D-ribitol + NAD+ = D-ribulose + H+ + NADH. Sources: EC:1.1.1.56, RHEA:20053 Also known as: adonitol dehydrogenase activity, ribitol dehydrogenase A (wild type), ribitol dehydrogenase B (mutant enzyme with different properties), ribitol dehydrogenase D (mutant enzyme with different properties), ribitol:NAD+ 2-oxidoreductase activity Relationships: is a type of oxidoreductase activity, acting on the CH-OH group of donors, NAD or NADP as acceptor [GO:0016616]